negative regulation of plasmacytoid dendritic cell antigen processing and presentation [GO:0002611] (biological process) Also known as: down regulation of plasmacytoid dendritic cell antigen processing and presentation, down-regulation of plasmacytoid dendritic cell antigen processing and presentation, downregulation of plasmacytoid dendritic cell antigen processing and presentation, inhibition of plasmacytoid dendritic cell antigen processing and presentation Definition: Any process that stops, prevents, or reduces the frequency, rate, or extent of plasmacytoid dendritic cell antigen processing and presentation. Sources: GOC:add Relationships: is a type of GO:0002605; is a type of regulation of plasmacytoid dendritic cell antigen processing and presentation [GO:0002610]; RO_0002212 plasmacytoid dendritic cell antigen processing and presentation [GO:0002470]